{
  "gene_name": "NHL-repeat-containing protein 4",
  "term_id": "UNKNOWN:0001",
  "term_label": "Unknown molecular function",
  "gene": "UniProtKB:P0CG21",
  "gene_symbol": "NHLRC4"
}